positive gravitropism [GO:0009958] (biological process) Definition: The orientation of plant parts towards gravity. Also known as: root gravitropism Sources: GOC:sm Relationships: is a type of GO:0009630